N6-methyl-AMP deaminase activity [GO:0062154] (molecular function) Definition: Catalysis of the reaction: H+ + H2O + N6-methyl-AMP = IMP + methylamine. Can also use N6-methyl-dAMP as a substrate. Also known as: MAPDA, N6-mAMP deaminase activity, N6-methyl-AMP/dAMP aminohydrolase Relationships: is_a GO:0019239 References: PMID:29884623 Sources: RHEA:16001